negative regulation of seed germination [GO:0010187] (biological process) Definition: Any process that stops, prevents, or reduces the frequency, rate or extent of seed germination. Sources: GOC:tb Also known as: down regulation of seed germination, down-regulation of seed germination, downregulation of seed germination, inhibition of seed germination Relationships: is a type of GO:0010029; is_a GO:0048581; negatively regulates seed germination [GO:0009845]